{
  "gene_symbol": "CNTNAP4",
  "gene": "UniProtKB:Q9C0A0",
  "term_label": "Unknown molecular function",
  "gene_name": "Contactin-associated protein-like 4",
  "term_id": "UNKNOWN:0001"
}